{
  "term_label": "Unknown molecular function",
  "gene_name": "Carcinoembryonic antigen-related cell adhesion molecule 5",
  "gene_symbol": "CEACAM5",
  "gene": "UniProtKB:P06731",
  "term_id": "UNKNOWN:0001"
}